axon choice point recognition [GO:0016198] (biological process) Subtypes: axon midline choice point recognition [GO:0016199] References: PMID:10218152 Relationships: is a type of neuron recognition [GO:0008038]; is part of axon guidance [GO:0007411] Definition: The recognition of molecules at a choice point by an axon growth cone; at a choice point the growth cone determines the direction of its future growth.